{
  "gene": "UniProtKB:P39023",
  "gene_symbol": "RPL3",
  "gene_name": "Large ribosomal subunit protein uL3",
  "term_id": "GO:0003723",
  "term_label": "RNA binding"
}